neural retina development [GO:0003407] (biological process) Regulation: regulated by regulation of neural retina development [GO:0061074]; positively regulated by positive regulation of neural retina development [GO:0061075]; negatively regulated by negative regulation of neural retina development [GO:0061076] Sources: GOC:ascb_2009, GOC:dph, GOC:tb Definition: The progression of the neural retina over time from its initial formation to the mature structure. The neural retina is the part of the retina that contains neurons and photoreceptor cells. Relationships: is a type of anatomical structure development [GO:0048856]; is part of retina development in camera-type eye [GO:0060041]